response to anion stress [GO:0072342] (biological process) Relationships: is a type of response to salt stress [GO:0009651] References: PMID:19641131 Sources: GOC:cvs Definition: Any process that results in a change in state or activity of a cell or an organism (in terms of movement, secretion, enzyme production, gene expression, etc.) as a result of anion stress, an increase or decrease in the concentration of negatively charged ions in the environment.